{
  "term_id": "GO:0098839",
  "gene": "UniProtKB:P42263",
  "gene_name": "Glutamate receptor 3",
  "term_label": "postsynaptic density membrane",
  "gene_symbol": "GRIA3"
}